{
  "gene": "UniProtKB:Q8TDY8",
  "gene_symbol": "IGDCC4",
  "term_id": "UNKNOWN:0003",
  "gene_name": "Immunoglobulin superfamily DCC subclass member 4",
  "term_label": "Unknown cellular component"
}